{
  "gene": "UniProtKB:Q8WZ69",
  "term_id": "UNKNOWN:0003",
  "gene_symbol": "C11orf40",
  "term_label": "Unknown cellular component",
  "gene_name": "Putative uncharacterized protein C11orf40"
}